muramyl dipeptide kinase activity [GO:0160047] (molecular function) Definition: Catalysis of the reaction: ATP + muramyl dipeptide = ADP + H+ + 6-O-phospho-muramyl dipeptide. References: PMID:36002575 Relationships: is a type of kinase activity [GO:0016301]